{
  "gene_name": "Junctional sarcoplasmic reticulum protein 1",
  "gene": "UniProtKB:Q96MG2",
  "gene_symbol": "JSRP1",
  "term_id": "GO:0003009",
  "term_label": "skeletal muscle contraction"
}